{
  "gene": "UniProtKB:Q5VZP5",
  "term_id": "GO:0005737",
  "gene_name": "Serine_threonine_tyrosine-interacting-like protein 2",
  "gene_symbol": "STYXL2",
  "term_label": "cytoplasm"
}